transferase activity, transferring phosphorus-containing groups [GO:0016772] (molecular function) Relationships: is a type of GO:0016740 Subtypes: kinase activity [GO:0016301], phosphotransferase activity, alcohol group as acceptor [GO:0016773], phosphotransferase activity, carboxyl group as acceptor [GO:0016774], phosphotransferase activity, nitrogenous group as acceptor [GO:0016775], phosphotransferase activity, phosphate group as acceptor [GO:0016776], GO:0016778, GO:0016779, phosphotransferase activity, for other substituted phosphate groups [GO:0016780], phosphotransferase activity, paired acceptors [GO:0016781], glycogen synthase activity, transferring glucose-1-phosphate [GO:0061547], ADP-riboxanase activity [GO:0140740] Note: Note that this term encompasses all kinase activities, as well as activities that transfer other phosphorus-containing groups such as diphosphate or nucleotides. Definition: Catalysis of the transfer of a phosphorus-containing group from one compound (donor) to another (acceptor). Sources: EC:2.7.-.-